{
  "term_label": "terminal bouton",
  "gene": "UniProtKB:O14795",
  "term_id": "GO:0043195",
  "gene_name": "Protein unc-13 homolog B",
  "gene_symbol": "UNC13B"
}